{
  "term_id": "GO:0006355",
  "gene_name": "SET-binding protein",
  "gene": "UniProtKB:Q9Y6X0",
  "gene_symbol": "SETBP1",
  "term_label": "regulation of DNA-templated transcription"
}